{
  "term_id": "UNKNOWN:0001",
  "gene": "UniProtKB:Q6ZSA8",
  "gene_symbol": "Q6ZSA8",
  "gene_name": "Putative uncharacterized protein FLJ45684",
  "term_label": "Unknown molecular function"
}